regulation of oxytocin production [GO:0140667] (biological process) Definition: Any process that modulates the frequency, rate, or extent of production of oxytocin. Subtypes: positive regulation of oxytocin production [GO:0140668], negative regulation of oxytocin production [GO:0140669] Relationships: is a type of regulation of gene expression [GO:0010468]; regulates oxytocin production [GO:0036162] References: PMID:25096581